{
  "gene_symbol": "S100A7A",
  "term_id": "GO:0043542",
  "term_label": "endothelial cell migration",
  "gene_name": "Protein S100-A7A",
  "gene": "UniProtKB:Q86SG5"
}